{
  "gene": "UniProtKB:A8MRT5",
  "gene_symbol": "NPIPB5",
  "term_label": "Unknown molecular function",
  "term_id": "UNKNOWN:0001",
  "gene_name": "Nuclear pore complex-interacting protein family member B5"
}